{
  "gene_name": "Retinal rod rhodopsin-sensitive cGMP 3',5'-cyclic phosphodiesterase subunit gamma",
  "gene": "UniProtKB:P18545",
  "gene_symbol": "PDE6G",
  "term_label": "Unknown molecular function",
  "term_id": "UNKNOWN:0001"
}